{
  "term_label": "eRF1 methyltransferase complex",
  "term_id": "GO:0035657",
  "gene": "UniProtKB:Q9Y5N5",
  "gene_symbol": "HEMK2",
  "gene_name": "Methyltransferase N6AMT1"
}